periciliary membrane compartment [GO:1990075] (cellular component) References: PMID:22342749 Sources: GOC:cilia, GOC:dr, GOC:krc Relationships: is a type of plasma membrane region [GO:0098590] Also known as: PCMC Definition: A plasma membrane region adjacent to the base of eukaryotic cilia and flagella that is enriched in endocytosis-associated proteins and vesicles and that appears to regulate ciliary membrane homeostasis.